{
  "term_id": "UNKNOWN:0002",
  "gene": "UniProtKB:A0A075B7E0",
  "gene_name": "Protein IGHD3OR15-3A (Fragment)",
  "gene_symbol": "IGHD3OR15-3B",
  "term_label": "Unknown biological process"
}